IgG B cell receptor complex [GO:0071737] (cellular component) Definition: An IgG immunoglobulin complex that is present in the plasma membrane of B cells and is composed of two identical immunoglobulin heavy chains of an IgG isotype and two identical immunoglobulin light chains and a signaling subunit, a heterodimer of the Ig-alpha and Ig-beta proteins. Sources: GOC:add, ISBN:0781765196 Also known as: membrane-bound IgG, membrane-bound IgG1, membrane-bound IgG2, membrane-bound IgG2a, membrane-bound IgG2b, membrane-bound IgG2c, membrane-bound IgG3, membrane-bound IgG4, surface IgG, surface IgG1, surface IgG2, surface IgG2a, surface IgG2b, surface IgG2c, surface IgG3, surface IgG4 Note: Note that an IgG immunoglobulin complex has the function of antigen binding if a suitable antigen is available. Also, IgG isotypes vary by species. Relationships: is a type of B cell receptor complex [GO:0019815]; is a type of GO:0071735